{
  "gene": "UniProtKB:Q9NP90",
  "gene_symbol": "RAB9B",
  "term_id": "GO:0005764",
  "gene_name": "Ras-related protein Rab-9B",
  "term_label": "lysosome"
}